establishment of protein localization to chromosome [GO:0070199] (biological process) Also known as: establishment of protein localisation to chromosome Subtypes: establishment of protein localization to telomere [GO:0070200], GO:0071169, protein transport along microtubule to kinetochore [GO:0140210] Definition: The directed movement of a protein to a specific location on a chromosome. Regulation: regulated by regulation of establishment of protein localization to chromosome [GO:0070202] Sources: GOC:BHF, GOC:mah Relationships: is a type of establishment of protein localization to organelle [GO:0072594]